{
  "gene_symbol": "SNRPGP15",
  "gene_name": "Putative small nuclear ribonucleoprotein G-like protein 15",
  "gene": "UniProtKB:A8MWD9",
  "term_id": "GO:0071013",
  "term_label": "catalytic step 2 spliceosome"
}